{
  "gene_symbol": "TRPA1",
  "gene_name": "Transient receptor potential cation channel subfamily A member 1",
  "term_id": "GO:0015278",
  "gene": "UniProtKB:O75762",
  "term_label": "intracellularly gated calcium channel activity"
}